{
  "gene": "UniProtKB:Q9Y426",
  "term_id": "UNKNOWN:0001",
  "gene_name": "C2 domain-containing protein 2",
  "term_label": "Unknown molecular function",
  "gene_symbol": "C2CD2"
}